{
  "gene_name": "Somatostatin",
  "term_label": "extracellular space",
  "gene": "UniProtKB:P61278",
  "term_id": "GO:0005615",
  "gene_symbol": "SST"
}